{
  "gene_name": "N-acetylglucosamine-6-sulfatase",
  "term_id": "GO:0005764",
  "gene_symbol": "GNS",
  "term_label": "lysosome",
  "gene": "UniProtKB:P15586"
}